{
  "gene_symbol": "NOL7",
  "gene_name": "Nucleolar protein 7",
  "gene": "UniProtKB:Q9UMY1",
  "term_id": "GO:0005730",
  "term_label": "nucleolus"
}